regulation of fumagillin biosynthetic process [GO:1902090] (biological process) Also known as: regulation of fumagillin anabolism, regulation of fumagillin biosynthesis, regulation of fumagillin formation, regulation of fumagillin synthesis Definition: Any process that modulates the frequency, rate or extent of fumagillin biosynthetic process. Subtypes: negative regulation of fumagillin biosynthetic process [GO:1902091], positive regulation of fumagillin biosynthetic process [GO:1902092] References: PMID:23488861 Sources: GOC:TermGenie, GOC:di Relationships: is a type of GO:0009889; is a type of GO:0043455; is a type of regulation of small molecule metabolic process [GO:0062012]; regulates fumagillin biosynthetic process [GO:1902086]